{
  "gene": "UniProtKB:P49006",
  "term_label": "plasma membrane",
  "gene_name": "MARCKS-related protein",
  "gene_symbol": "MARCKSL1",
  "term_id": "GO:0005886"
}